{
  "term_label": "Unknown molecular function",
  "gene": "UniProtKB:P78312",
  "gene_symbol": "FAM193A",
  "gene_name": "Protein FAM193A",
  "term_id": "UNKNOWN:0001"
}